{
  "term_id": "GO:0005634",
  "gene_symbol": "KDM5A",
  "gene_name": "Lysine-specific demethylase 5A",
  "gene": "UniProtKB:P29375",
  "term_label": "nucleus"
}